microtubule anchoring at microtubule organizing center [GO:0072393] (biological process) Definition: Any process in which a microtubule is maintained in a specific location in a cell by attachment to a microtubule organizing center. References: PMID:19825938 Sources: GOC:BHF Also known as: microtubule anchoring at MTOC, microtubule anchoring at microtubule organising centre Relationships: is a type of microtubule anchoring [GO:0034453] Subtypes: microtubule anchoring at centrosome [GO:0034454], microtubule anchoring at spindle pole body [GO:0034631]